(R)-lactaldehyde dehydrogenase activity [GO:0102641] (molecular function) Sources: GOC:pz Definition: Catalysis of the reaction: (R)-propane-1,2-diol + NADP = (R)-lactaldehyde + NADPH + H+. Relationships: is a type of oxidoreductase activity, acting on the CH-OH group of donors, NAD or NADP as acceptor [GO:0016616]